regulation of organelle transport along microtubule [GO:1902513] (biological process) References: PMID:21147087 Sources: GOC:TermGenie, GOC:dph Subtypes: regulation of anterograde axonal transport of mitochondrion [GO:0061880], GO:1901608, GO:1902838 Definition: Any process that modulates the frequency, rate or extent of organelle transport along microtubule. Relationships: is a type of regulation of intracellular transport [GO:0032386]; is a type of GO:0060632; regulates organelle transport along microtubule [GO:0072384] Also known as: regulation of microtubule-based organelle localization